{
  "term_label": "neutral amino acid transport",
  "gene": "UniProtKB:O75387",
  "gene_name": "Large neutral amino acids transporter small subunit 3",
  "gene_symbol": "SLC43A1",
  "term_id": "GO:0015804"
}